{
  "gene_symbol": "MRPS17",
  "gene": "UniProtKB:Q9Y2R5",
  "gene_name": "Small ribosomal subunit protein uS17m",
  "term_label": "Unknown biological process",
  "term_id": "UNKNOWN:0002"
}